negative regulation of delayed rectifier potassium channel activity [GO:1902260] (biological process) References: PMID:11299204 Sources: GOC:BHF, GOC:TermGenie, GOC:mtg_cardiac_conduct_nov11, GOC:rl Definition: Any process that stops, prevents or reduces the frequency, rate or extent of delayed rectifier potassium channel activity. Also known as: down regulation of delayed rectifier potassium channel activity, down-regulation of delayed rectifier potassium channel activity, downregulation of delayed rectifier potassium channel activity, inhibition of delayed rectifier potassium channel activity Relationships: is a type of regulation of delayed rectifier potassium channel activity [GO:1902259]; is a type of negative regulation of voltage-gated potassium channel activity [GO:1903817]; negatively regulates delayed rectifier potassium channel activity [GO:0005251]